alanine-tRNA ligase activity [GO:0004813] (molecular function) Sources: EC:6.1.1.7 Definition: Catalysis of the reaction: ATP + L-alanine + tRNA(Ala) = AMP + diphosphate + L-alanyl-tRNA(Ala). Relationships: is a type of aminoacyl-tRNA ligase activity [GO:0004812] Also known as: alanyl-tRNA synthetase activity, Ala-tRNA synthetase activity, AlaRS, L-alanine:tRNAAla ligase (AMP-forming), alanine tRNA synthetase activity, alanine transfer RNA synthetase activity, alanine translase activity, alanine-transfer RNA ligase activity, alanyl-transfer RNA synthetase activity, alanyl-transfer ribonucleate synthase activity, alanyl-transfer ribonucleate synthetase activity, alanyl-transfer ribonucleic acid synthetase activity